ameboidal-type cell migration [GO:0001667] (biological process) Definition: Cell migration that is accomplished by extension and retraction of a pseudopodium. Relationships: is_a cell migration [GO:0016477] Subtypes: mesodermal cell migration [GO:0008078], epithelial cell migration [GO:0010631], fibroblast migration [GO:0010761], cell migration involved in gastrulation [GO:0042074], trophoblast cell migration [GO:0061450], GO:0090497 Note: Note that this term refers to a mode of migration rather than to any particular cell type. Also known as: ameboid cell migration, amoeboid cell migration, amoeboidal cell migration Sources: GOC:dph